{
  "term_label": "metalloendopeptidase activity",
  "gene_symbol": "OMA1",
  "term_id": "GO:0004222",
  "gene": "UniProtKB:Q96E52",
  "gene_name": "Metalloendopeptidase OMA1, mitochondrial"
}